{
  "gene_symbol": "DEFB4B",
  "term_label": "chemoattractant activity",
  "gene": "UniProtKB:O15263",
  "term_id": "GO:0042056",
  "gene_name": "Defensin beta 4A"
}